{
  "term_id": "GO:0042800",
  "term_label": "histone H3K4 methyltransferase activity",
  "gene_symbol": "SETD1A",
  "gene": "UniProtKB:O15047",
  "gene_name": "Histone-lysine N-methyltransferase SETD1A"
}